transferrin transport [GO:0033572] (biological process) Also known as: melanotransferrin transport Sources: GOC:mlg Definition: The directed movement of transferrin into, out of or within a cell, or between cells, by means of some agent such as a transporter or pore. Relationships: is a type of iron ion transport [GO:0006826]; is_a protein transport [GO:0015031]